prostaglandin receptor activity [GO:0004955] (molecular function) Definition: Combining with a prostaglandin (PG) to initiate a change in cell activity. Sources: ISBN:0198506732 Relationships: is a type of prostanoid receptor activity [GO:0004954] Subtypes: prostaglandin J receptor activity [GO:0001785], prostaglandin D receptor activity [GO:0004956], prostaglandin E receptor activity [GO:0004957], prostaglandin F receptor activity [GO:0004958], GO:0016501